{
  "gene": "UniProtKB:Q9Y6R6",
  "term_id": "GO:0001228",
  "gene_name": "Zinc finger protein 780B",
  "term_label": "DNA-binding transcription activator activity, RNA polymerase II-specific",
  "gene_symbol": "ZNF780B"
}